cochlea development [GO:0090102] (biological process) Sources: GOC:dph, GOC:tb Relationships: is a type of anatomical structure development [GO:0048856]; is part of GO:0048839 Definition: The progression of the cochlea over time from its formation to the mature structure. The cochlea is the snail-shaped portion of the inner ear that is responsible for the detection of sound.